regulation of ryanodine-sensitive calcium-release channel activity [GO:0060314] (BP) Definition: Any process that modulates the activity of a ryanodine-sensitive calcium-release channel. The ryanodine-sensitive calcium-release channel catalyzes the transmembrane transfer of a calcium ion by a channel that opens when a ryanodine class ligand has been bound by the channel complex or one of its constituent parts. Sources: GOC:BHF, GOC:dph, GOC:tb Relationships: is a type of regulation of transmembrane transporter activity [GO:0022898]; is a type of GO:0051279; regulates ryanodine-sensitive calcium-release channel activity [GO:0005219] Subtypes: negative regulation of ryanodine-sensitive calcium-release channel activity [GO:0060315]